{
  "gene": "UniProtKB:P0C628",
  "gene_symbol": "OR5AC1",
  "gene_name": "Olfactory receptor 5AC1",
  "term_id": "GO:0005549",
  "term_label": "odorant binding"
}